{
  "gene_symbol": "ERC2",
  "gene": "UniProtKB:O15083",
  "term_id": "GO:0098831",
  "term_label": "presynaptic active zone cytoplasmic component",
  "gene_name": "ERC protein 2"
}